rRNA (uridine) methyltransferase activity [GO:0016436] (molecular function) Definition: Catalysis of the reaction: S-adenosyl-L-methionine + rRNA = S-adenosyl-L-homocysteine + rRNA containing methyluridine. Relationships: is a type of rRNA methyltransferase activity [GO:0008649] Sources: GOC:go-curators Subtypes: GO:0008650, GO:0070041, GO:0070042